{
  "gene_name": "F-BAR and double SH3 domains protein 2",
  "term_id": "GO:0055037",
  "gene_symbol": "FCHSD2",
  "term_label": "recycling endosome",
  "gene": "UniProtKB:O94868"
}